{
  "gene_name": "Gastrin-releasing peptide",
  "term_id": "GO:2000987",
  "gene": "UniProtKB:P07492",
  "gene_symbol": "GRP",
  "term_label": "positive regulation of behavioral fear response"
}